3-phenylpropionate catabolic process [GO:0019380] (biological process) Definition: The chemical reactions and pathways resulting in the breakdown of 3-phenylpropionate, the anion of phenylpropanoic acid. Sources: GOC:ai Also known as: 3-phenylpropionate breakdown, 3-phenylpropionate catabolism, 3-phenylpropionate degradation Relationships: is a type of xenobiotic catabolic process [GO:0042178]; is a type of benzene-containing compound metabolic process [GO:0042537]; is a type of monocarboxylic acid catabolic process [GO:0072329]